{
  "gene": "UniProtKB:Q969H8",
  "gene_symbol": "MYDGF",
  "term_id": "UNKNOWN:0001",
  "gene_name": "Myeloid-derived growth factor",
  "term_label": "Unknown molecular function"
}